{
  "term_label": "RNA polymerase II transcription regulatory region sequence-specific DNA binding",
  "gene_symbol": "RHOXF1",
  "term_id": "GO:0000977",
  "gene": "UniProtKB:Q8NHV9",
  "gene_name": "Rhox homeobox family member 1"
}